{
  "gene_symbol": "STAT5A",
  "term_label": "cytoplasm",
  "gene_name": "Signal transducer and activator of transcription 5A",
  "term_id": "GO:0005737",
  "gene": "UniProtKB:P42229"
}